{
  "term_id": "GO:0016592",
  "term_label": "mediator complex",
  "gene_symbol": "MED31",
  "gene": "UniProtKB:Q9Y3C7",
  "gene_name": "Mediator of RNA polymerase II transcription subunit 31"
}